L-cysteine desulfhydrase activity [GO:0080146] (molecular function) Definition: Catalysis of the reaction: L-cysteine + H2O = ammonia + pyruvate + hydrogen sulfide + H+. References: PMID:19955263 Sources: MetaCyc:LCYSDESULF-RXN Relationships: is a type of carbon-sulfur lyase activity [GO:0016846]